{
  "gene_name": "Histone-lysine N-methyltransferase EZH2",
  "gene_symbol": "EZH2",
  "term_id": "GO:0005634",
  "gene": "UniProtKB:Q15910",
  "term_label": "nucleus"
}